{
  "gene_name": "NADH dehydrogenase [ubiquinone] 1 beta subcomplex subunit 5, mitochondrial",
  "term_label": "respiratory chain complex I",
  "gene_symbol": "NDUFB5",
  "gene": "UniProtKB:O43674",
  "term_id": "GO:0045271"
}